{
  "term_id": "GO:0051123",
  "gene_symbol": "TAF11L13",
  "gene": "UniProtKB:A0A1W2PPH5",
  "term_label": "RNA polymerase II preinitiation complex assembly",
  "gene_name": "TATA-box-binding protein-associated factor 11-like protein 13"
}